maintenance of dormancy [GO:0097437] (biological process) Relationships: is a type of dormancy process [GO:0022611] Subtypes: maintenance of seed dormancy [GO:0010231] Definition: The dormancy process that results in an organism remaining in dormancy. Dormancy (sometimes called a dormant state) is a suspension of most physiological activity and growth that can be reactivated. Sources: GOC:PO_curators, PO_REF:00009